{
  "gene": "UniProtKB:A0A286YEV6",
  "gene_name": "Small cysteine and glycine repeat-containing protein 4",
  "term_label": "Unknown cellular component",
  "term_id": "UNKNOWN:0003",
  "gene_symbol": "SCYGR4"
}